3-ethylmalate synthase activity [GO:0050441] (molecular function) Sources: RHEA:10500 Also known as: 2-ethyl-3-hydroxybutanedioate synthase activity, 3-ethylmalate glyoxylate-lyase (CoA-butanoylating) activity, butanoyl-CoA:glyoxylate C-butanoyltransferase (thioester-hydrolysing, 1-carboxypropyl-forming) Relationships: is a type of acyltransferase activity, acyl groups converted into alkyl on transfer [GO:0046912] Definition: Catalysis of the reaction: butanoyl-CoA + glyoxylate + H2O = 3-ethylmalate + CoA + H+.